16-hydroxypalmitate dehydrogenase activity [GO:0103002] (molecular function) Definition: Catalysis of the reaction: 16-hydroxypalmitate + NADP = H+ + 16-oxo-palmitate + NADPH. Relationships: is a type of oxidoreductase activity, acting on the CH-OH group of donors, NAD or NADP as acceptor [GO:0016616] Sources: GOC:pz